{
  "term_label": "clathrin-dependent endocytosis",
  "gene_name": "Growth arrest-specific protein 7",
  "term_id": "GO:0072583",
  "gene": "UniProtKB:O60861",
  "gene_symbol": "GAS7"
}